{
  "term_label": "cytoplasm",
  "gene": "UniProtKB:P23508",
  "term_id": "GO:0005737",
  "gene_symbol": "MCC",
  "gene_name": "Colorectal mutant cancer protein"
}